{
  "term_label": "very long-chain fatty acid biosynthetic process",
  "gene_name": "Very-long-chain (3R)-3-hydroxyacyl-CoA dehydratase 1",
  "term_id": "GO:0042761",
  "gene_symbol": "HACD1",
  "gene": "UniProtKB:B0YJ81"
}